negative regulation of dopaminergic neuron differentiation [GO:1904339] (biological process) References: PMID:15522889 Sources: GOC:TermGenie, GO_REF:0000058 Subtypes: GO:1904957 Also known as: down regulation of dopaminergic neuron differentiation, down-regulation of dopaminergic neuron differentiation, downregulation of dopaminergic neuron differentiation, inhibition of dopaminergic neuron differentiation Definition: Any process that stops, prevents or reduces the frequency, rate or extent of dopaminergic neuron differentiation. Relationships: is a type of negative regulation of neuron differentiation [GO:0045665]; is a type of regulation of dopaminergic neuron differentiation [GO:1904338]; negatively regulates GO:0071542